{
  "gene_symbol": "AGXT2",
  "term_label": "L-alanine catabolic process, by transamination",
  "gene_name": "Alanine--glyoxylate aminotransferase 2, mitochondrial",
  "gene": "UniProtKB:Q9BYV1",
  "term_id": "GO:0019481"
}